mitotic metaphase chromosome recapture [GO:1990942] (biological process) Definition: A mechanism to recapture 'lost' chromosomes (chromosomes which have become detached from the spindle) during metaphase of mitotic chromosome segregation. Chromosomes with unattached kinetochores are migrated along (non polar) spindle microtubules to the mitotic spindle pole body by a combination of microtubule depolymerisation and 'kinetochore sliding' (migration of the chromosome along the microtubule). The chromosome subsequently migrates along the polar spindle microtubule to the metaphase plate. Relationships: is a type of chromosome localization [GO:0050000]; is part of GO:0007080 Also known as: kinetochore retrieval, metaphase chromosome retrieval to the spindle pole body, microtubule sliding involved in kinetochore retrieval, microtubule sliding involved in metaphase chromosome retrieval to the spindle pole body, microtubule sliding involved in sister kinetochore recapture, sister kinetochore recapture, microtubule sliding involved in mitotic metaphase chromosome recapture References: PMID:18256284